{
  "gene": "UniProtKB:Q9HB19",
  "gene_symbol": "PLEKHA2",
  "gene_name": "Pleckstrin homology domain-containing family A member 2",
  "term_label": "phosphatidylinositol-3,4-bisphosphate binding",
  "term_id": "GO:0043325"
}